{
  "gene": "UniProtKB:Q7RTT6",
  "term_label": "nucleus",
  "gene_name": "Putative protein SSX6",
  "term_id": "GO:0005634",
  "gene_symbol": "SSX6P"
}